{
  "gene": "UniProtKB:Q9UPR3",
  "term_label": "telomerase RNA binding",
  "gene_symbol": "SMG5",
  "gene_name": "Nonsense-mediated mRNA decay factor SMG5",
  "term_id": "GO:0070034"
}